CNBH domain intrinsic ligand binding [GO:0106151] (molecular function) Definition: Interacting selectivity and noncovalently with a cyclic nucleotide mimicking protein motif that is part of the same protein. The CNBHD is a domain on KCNH channels that creates a binding pocket on the KCNH channel that resembles the cyclic nucleotide- binding domain on other ion channels. It binds to a peptide motif that is part of the same protein rather than a cyclic nucleotide. Relationships: is a type of GO:0005515 References: PMID:27025590, PMID:29567795 Sources: GOC:cvs Note: It is unclear if the motif bound by CNBHD is a specific motif or just a beta sheet with the appropriate amino acids.